petromyzonol sulfotransferase activity [GO:0033873] (molecular function) Definition: Catalysis of the reaction: 3'-phospho-5'-adenylyl sulfate + 5alpha-cholane-3alpha,7alpha,12alpha,24-tetrol = 3alpha,7alpha,12alpha-trihydroxy-5alpha-cholan-24-yl sulfate + adenosine 3',5'-diphosphate + H+. Sources: EC:2.8.2.31, RHEA:16997 Also known as: 3'-phosphoadenylyl-sulfate:5alpha-cholan-3alpha,7alpha,12alpha,24-tetrol sulfotransferase activity, PZ-SULT Relationships: is a type of sulfotransferase activity [GO:0008146]